{
  "term_label": "axoneme",
  "gene_symbol": "DYDC1",
  "gene_name": "DPY30 domain-containing protein 1",
  "gene": "UniProtKB:Q8WWB3",
  "term_id": "GO:0005930"
}